{
  "gene_name": "Protein BEX2",
  "gene": "UniProtKB:Q9BXY8",
  "gene_symbol": "BEX2",
  "term_label": "cytoplasm",
  "term_id": "GO:0005737"
}